fatty acyl-CoA hydrolase activity [GO:0047617] (molecular function) Definition: Catalysis of the reaction: a fatty acyl-CoA + H2O = a fatty acid + CoA + H+. Relationships: is a type of acyl-CoA hydrolase activity [GO:0016289] Also known as: acyl-CoA hydrolase activity, acyl-CoA thioesterase activity, acyl-CoA thiolesterase activity, acyl-CoA thioesterase I activity, acyl-CoA thioesterase II activity, acyl coenzyme A hydrolase activity, acyl coenzyme A thioesterase activity, thioesterase B, thioesterase II Subtypes: medium-chain fatty acyl-CoA hydrolase activity [GO:0052815], GO:0052816, very long-chain fatty acyl-CoA hydrolase activity [GO:0052817], short-chain fatty acyl-CoA hydrolase activity [GO:0141126] Sources: RHEA:16781